{
  "term_label": "Unknown cellular component",
  "gene": "UniProtKB:Q96GT9",
  "gene_symbol": "XAGE2",
  "gene_name": "X antigen family member 2",
  "term_id": "UNKNOWN:0003"
}